{
  "gene": "UniProtKB:P34059",
  "gene_name": "N-acetylgalactosamine-6-sulfatase",
  "term_label": "arylsulfatase activity",
  "gene_symbol": "GALNS",
  "term_id": "GO:0004065"
}